{
  "term_label": "Unknown molecular function",
  "term_id": "UNKNOWN:0001",
  "gene": "UniProtKB:P25189",
  "gene_name": "Myelin protein P0",
  "gene_symbol": "MPZ"
}